{
  "term_id": "GO:0019158",
  "gene_symbol": "GCK",
  "gene": "UniProtKB:P35557",
  "gene_name": "Hexokinase-4",
  "term_label": "mannokinase activity"
}